{
  "gene_symbol": "DDIT4",
  "gene_name": "DNA damage-inducible transcript 4 protein",
  "term_id": "GO:0006915",
  "term_label": "apoptotic process",
  "gene": "UniProtKB:Q9NX09"
}